{
  "gene": "UniProtKB:Q96EP5",
  "gene_symbol": "DAZAP1",
  "term_id": "GO:0005634",
  "term_label": "nucleus",
  "gene_name": "DAZ-associated protein 1"
}